{
  "gene_name": "Prostaglandin E synthase 2",
  "gene": "UniProtKB:Q9H7Z7",
  "term_label": "mitochondrion",
  "term_id": "GO:0005739",
  "gene_symbol": "PTGES2"
}